{
  "gene_symbol": "C1QTNF5",
  "term_label": "extracellular space",
  "term_id": "GO:0005615",
  "gene": "UniProtKB:Q9BXJ0",
  "gene_name": "Complement C1q tumor necrosis factor-related protein 5"
}